{
  "gene": "UniProtKB:O60296",
  "gene_name": "Trafficking kinesin-binding protein 2",
  "term_id": "GO:0050811",
  "gene_symbol": "TRAK2",
  "term_label": "GABA receptor binding"
}